{
  "gene": "UniProtKB:P0CG34",
  "gene_name": "Thymosin beta-15A",
  "term_id": "GO:0030334",
  "term_label": "regulation of cell migration",
  "gene_symbol": "TMSB15A"
}